late endosome to lysosome transport [GO:1902774] (biological process) Regulation: regulated by regulation of late endosome to lysosome transport [GO:1902822]; negatively regulated by negative regulation of late endosome to lysosome transport [GO:1902823]; positively regulated by positive regulation of late endosome to lysosome transport [GO:1902824] Note: an example of this is snapin in mouse (Q9Z266) in PMID:20920792 inferred from mutant phenotype References: PMID:23949442 Sources: GOC:TermGenie, GO_REF:0000076 Relationships: is a type of lysosomal transport [GO:0007041] Definition: The directed movement of substances from late endosome to lysosome. Also known as: prevacuolar compartment to lysosome transport Subtypes: GO:0061764